{
  "gene_name": "Cyclic AMP-dependent transcription factor ATF-5",
  "term_label": "nucleus",
  "gene": "UniProtKB:Q9Y2D1",
  "term_id": "GO:0005634",
  "gene_symbol": "ATF5"
}